{
  "term_label": "DNA-binding transcription factor activity, RNA polymerase II-specific",
  "gene": "UniProtKB:P14921",
  "term_id": "GO:0000981",
  "gene_name": "Protein C-ets-1",
  "gene_symbol": "ETS1"
}